{
  "gene_symbol": "ZNF385A",
  "term_label": "neuronal cell body",
  "gene": "UniProtKB:Q96PM9",
  "term_id": "GO:0043025",
  "gene_name": "Zinc finger protein 385A"
}